{
  "gene_name": "Cellular retinoic acid-binding protein 1",
  "term_id": "GO:0005829",
  "gene_symbol": "CRABP1",
  "term_label": "cytosol",
  "gene": "UniProtKB:P29762"
}